positive regulation of glial cell apoptotic process [GO:0034352] (biological process) Also known as: up regulation of glial cell apoptosis, up-regulation of glial cell apoptosis, upregulation of glial cell apoptosis, activation of glial cell apoptosis, positive regulation of glial cell apoptosis, stimulation of glial cell apoptosis Definition: Any process that activates or increases the frequency, rate, or extent of glial cell apoptotic process. Subtypes: positive regulation of oligodendrocyte apoptotic process [GO:1900143] Sources: GOC:mah, GOC:mtg_apoptosis Relationships: is a type of regulation of glial cell apoptotic process [GO:0034350]; is_a positive regulation of apoptotic process [GO:0043065]; positively regulates glial cell apoptotic process [GO:0034349]